{
  "term_id": "GO:0004869",
  "gene": "UniProtKB:P01036",
  "gene_symbol": "CST4",
  "gene_name": "Cystatin-S",
  "term_label": "cysteine-type endopeptidase inhibitor activity"
}